{
  "gene_name": "Treslin",
  "term_label": "chromatin binding",
  "gene": "UniProtKB:Q7Z2Z1",
  "gene_symbol": "TICRR",
  "term_id": "GO:0003682"
}